{
  "gene_symbol": "NUP50",
  "gene_name": "Nuclear pore complex protein Nup50",
  "term_id": "UNKNOWN:0001",
  "term_label": "Unknown molecular function",
  "gene": "UniProtKB:Q9UKX7"
}